skein-like inclusion [GO:0097420] (cellular component) References: PMID:18026741 Sources: NIF_Subcellular:nlx_subcell_20090103 Relationships: is a type of inclusion body [GO:0016234] Definition: Intracytoplasmic filamentous structure frequently encountered in preparations immunostained for ubiquitin.